{
  "gene": "UniProtKB:A6NL99",
  "gene_symbol": "AQP7P3",
  "term_label": "Unknown cellular component",
  "gene_name": "Putative aquaporin-7-like protein 3",
  "term_id": "UNKNOWN:0003"
}